positive regulation of neural crest cell fate specification [GO:1905297] (biological process) Also known as: up regulation of neural crest cell fate specification, up-regulation of neural crest cell fate specification, upregulation of neural crest cell fate specification, activation of neural crest cell fate specification Relationships: is a type of positive regulation of cell fate specification [GO:0042660]; is a type of positive regulation of neural crest formation [GO:0090300]; is a type of positive regulation of neural crest cell differentiation [GO:1905294]; is a type of GO:1905295; positively regulates neural crest cell fate specification [GO:0014036] References: PMID:15073157 Sources: GOC:BHF, GOC:TermGenie, GOC:rl, GO_REF:0000058 Definition: Any process that activates or increases the frequency, rate or extent of neural crest cell fate specification.